Hechtian strand [GO:0120307] (cellular component) References: PMID:32397402 Sources: GOC:krc Relationships: is_a cellular anatomical structure [GO:0110165] Definition: An extended membranous thread which firmly connects the plasma membrane to the cell wall during plasmolysis such that the plasma membrane does not separate from the cell wall completely.